{
  "term_id": "GO:0016251",
  "gene": "UniProtKB:A0A1W2PR64",
  "gene_symbol": "TAF11L9",
  "term_label": "RNA polymerase II general transcription initiation factor activity",
  "gene_name": "TATA-box-binding protein-associated factor 11-like protein 9"
}